{
  "gene_symbol": "TEFM",
  "term_label": "Unknown biological process",
  "gene_name": "Transcription elongation factor, mitochondrial",
  "term_id": "UNKNOWN:0002",
  "gene": "UniProtKB:Q96QE5"
}